tyrosine 3-monooxygenase activity [GO:0004511] (molecular function) Also known as: tyrosine 3-hydroxylase activity, tyrosine hydroxylase activity, L-tyrosine hydroxylase activity, L-tyrosine,tetrahydrobiopterin:oxygen oxidoreductase (3-hydroxylating) Definition: Catalysis of the reaction: L-tyrosine + tetrahydrobiopterin + O2 = 3,4-dihydroxy-L-phenylalanine + 4-alpha-hydroxytetrahydrobiopterin + H2O. Relationships: is a type of oxidoreductase activity, acting on paired donors, with incorporation or reduction of molecular oxygen, reduced pteridine as one donor, and incorporation of one atom of oxygen [GO:0016714] Regulation: positively regulated by GO:0036470 Sources: EC:1.14.16.2